phytochrome binding [GO:0010313] (molecular function) References: PMID:15486102 Relationships: is a type of GO:0005515 Definition: Binding to a phytochrome.